{
  "gene_symbol": "PIP4K2C",
  "term_id": "GO:0016309",
  "gene_name": "Phosphatidylinositol 5-phosphate 4-kinase type-2 gamma",
  "gene": "UniProtKB:Q8TBX8",
  "term_label": "1-phosphatidylinositol-5-phosphate 4-kinase activity"
}